{
  "gene_symbol": "AK3",
  "term_label": "cytoplasm",
  "gene": "UniProtKB:Q9UIJ7",
  "term_id": "GO:0005737",
  "gene_name": "GTP:AMP phosphotransferase AK3, mitochondrial"
}